{
  "term_id": "GO:0006906",
  "gene_name": "Synaptotagmin-11",
  "term_label": "vesicle fusion",
  "gene_symbol": "SYT11",
  "gene": "UniProtKB:Q9BT88"
}